{
  "term_id": "UNKNOWN:0002",
  "gene": "UniProtKB:Q6PCE3",
  "term_label": "Unknown biological process",
  "gene_name": "Glucose 1,6-bisphosphate synthase",
  "gene_symbol": "PGM2L1"
}